{
  "term_id": "GO:0005109",
  "gene_symbol": "BAMBI",
  "term_label": "frizzled binding",
  "gene": "UniProtKB:Q13145",
  "gene_name": "BMP and activin membrane-bound inhibitor homolog"
}